{
  "gene_symbol": "MEIOC",
  "gene_name": "Meiosis-specific coiled-coil domain-containing protein MEIOC",
  "gene": "UniProtKB:A2RUB1",
  "term_id": "GO:0005634",
  "term_label": "nucleus"
}